{
  "gene_name": "Syntaxin-binding protein 3",
  "term_id": "GO:0006886",
  "gene": "UniProtKB:O00186",
  "gene_symbol": "STXBP3",
  "term_label": "intracellular protein transport"
}